carboxylic acid biosynthetic process [GO:0046394] (biological process) Definition: The chemical reactions and pathways resulting in the formation of carboxylic acids, any organic acid containing one or more carboxyl (-COOH) groups. Sources: ISBN:0198506732 Also known as: carboxylic acid anabolism, carboxylic acid biosynthesis, carboxylic acid formation, carboxylic acid synthesis Relationships: is a type of organic acid biosynthetic process [GO:0016053]; is_a carboxylic acid metabolic process [GO:0019752] Subtypes: sulfur amino acid biosynthetic process [GO:0000097], amino acid catabolic process to carboxylic acid via Ehrlich pathway [GO:0000948], UDP-glucuronate biosynthetic process [GO:0006065], GO:0006780, GO:0009073, branched-chain amino acid biosynthetic process [GO:0009082], gibberellin biosynthetic process [GO:0009686], GO:0019289, GO:0019294, GO:0019853, oxylipin biosynthetic process [GO:0031408], L-homomethionine biosynthetic process [GO:0033322], carnosine biosynthetic process [GO:0035499], GO:0042121, GO:0042858, achromobactin biosynthetic process [GO:0042861], GO:0042864, dicarboxylic acid biosynthetic process [GO:0043650], GO:0046380, icosanoid biosynthetic process [GO:0046456], mannosylglycerate biosynthetic process [GO:0051479], GO:0071793, monocarboxylic acid biosynthetic process [GO:0072330], GO:0072351, GO:0170038, non-proteinogenic amino acid biosynthetic process [GO:0170043], GO:1900541, GO:1900578, endocrocin biosynthetic process [GO:1900602], GO:1900608, cspyrone B1 biosynthetic process [GO:1900802], helvolic acid biosynthetic process [GO:1900812], monodictyphenone biosynthetic process [GO:1900815], GO:1900870, cephalosporin C biosynthetic process [GO:1901268], GO:1901282, alpha-amino acid biosynthetic process [GO:1901607], GO:1901730